macrolide biosynthetic process [GO:0033068] (BP) Definition: The chemical reactions and pathways leading to the formation of macrolides, any of a large group of polyketide compounds that contain a large lactone ring with few or no double bonds and no nitrogen atoms, linked glycosidically to one or more sugar groups. The macrolides include the carbomycins, the erythromycins, oleandomycin, oligomycins, and the spiramycins, and act as antibiotics, mainly against Gram-positive bacteria. References: PMID:17298179 Sources: ISBN:0198506732 Also known as: macrolide anabolism, macrolide biosynthesis, macrolide formation, macrolide synthesis Subtypes: enterobactin biosynthetic process [GO:0009239], epothilone biosynthetic process [GO:0050814], GO:0106150, erythromycin biosynthetic process [GO:1901115] Relationships: is a type of GO:0017000; is a type of polyketide biosynthetic process [GO:0030639]; is_a macrolide metabolic process [GO:0033067]; is a type of lactone biosynthetic process [GO:1901336]